{
  "term_id": "GO:0007186",
  "gene_name": "Phosphatidylinositol 3,4,5-trisphosphate-dependent Rac exchanger 2 protein",
  "term_label": "G protein-coupled receptor signaling pathway",
  "gene_symbol": "PREX2",
  "gene": "UniProtKB:Q70Z35"
}